{
  "gene": "UniProtKB:P15923",
  "term_label": "chromatin",
  "term_id": "GO:0000785",
  "gene_symbol": "TCF3",
  "gene_name": "Transcription factor E2-alpha"
}